{
  "gene_name": "Adhesion G protein-coupled receptor E2",
  "gene_symbol": "ADGRE2",
  "gene": "UniProtKB:Q9UHX3",
  "term_label": "plasma membrane",
  "term_id": "GO:0005886"
}